(+)-taxifolin 5'-hydroxylase activity [GO:0102405] (molecular function) Definition: Catalysis of the reaction: (+)-taxifolin(1-) + O2 + NADPH(4-) + H+ = (+)-dihydromyricetin + NADP(3-) + H2O. Sources: GOC:pz Relationships: is a type of oxidoreductase activity, acting on paired donors, with incorporation or reduction of molecular oxygen, NAD(P)H as one donor, and incorporation of one atom of oxygen [GO:0016709]